{
  "gene_symbol": "SHCBP1",
  "gene": "UniProtKB:Q8NEM2",
  "term_label": "fibroblast growth factor receptor signaling pathway",
  "gene_name": "SHC SH2 domain-binding protein 1",
  "term_id": "GO:0008543"
}